{
  "gene_symbol": "OR13C5",
  "term_id": "GO:0004984",
  "gene_name": "Olfactory receptor 13C5",
  "term_label": "olfactory receptor activity",
  "gene": "UniProtKB:Q8NGS8"
}